diarylpropane peroxidase activity [GO:0016690] (molecular function) Also known as: LiP activity, ligninase I activity, 1,2-bis(3,4-dimethoxyphenyl)propane-1,3-diol:hydrogen-peroxide oxidoreductase activity, diarylpropane oxygenase activity, diarylpropane:oxygen,hydrogen-peroxide oxidoreductase (C-C-bond-cleaving), lignin peroxidase activity, ligninase activity Definition: Catalysis of the reaction: (3,4-dimethoxyphenyl)methanol + H2O2 = 3,4-dimethoxybenzaldehyde + 2 H2O. Relationships: is a type of peroxidase activity [GO:0004601] Sources: EC:1.11.1.14